regulation of cellodextrin catabolic process [GO:2000927] (biological process) Relationships: is a type of GO:0032881; is a type of regulation of carbohydrate catabolic process [GO:0043470]; regulates cellodextrin catabolic process [GO:2000890] Definition: Any process that modulates the frequency, rate or extent of cellodextrin catabolic process. Also known as: regulation of cellodextrin catabolism Sources: GOC:mengo_curators Subtypes: negative regulation of cellodextrin catabolic process [GO:2000928], positive regulation of cellodextrin catabolic process [GO:2000929]